{
  "gene_symbol": "ANO7",
  "gene": "UniProtKB:Q6IWH7",
  "term_label": "plasma membrane",
  "gene_name": "Anoctamin-7",
  "term_id": "GO:0005886"
}